establishment of organelle localization [GO:0051656] (biological process) Relationships: is a type of GO:0051234; is a type of organelle localization [GO:0051640] Definition: The directed movement of an organelle to a specific location. Also known as: establishment of organelle localisation Sources: GOC:ai Subtypes: ribosomal subunit export from nucleus [GO:0000054], nuclear migration [GO:0007097], GO:0043303, establishment of spindle localization [GO:0051293], establishment of vesicle localization [GO:0051650], establishment of mitochondrion localization [GO:0051654], establishment of centrosome localization [GO:0051660], establishment of plastid localization [GO:0051667], GO:0051683, establishment of ER localization [GO:0051686], organelle transport along microtubule [GO:0072384], microtubule plus-end directed mitotic chromosome migration [GO:0099606], autophagosome-dependent secretion [GO:0160192]